cytoskeletal anchor activity [GO:0008093] (molecular function) Definition: The binding activity of a protein that brings together a cytoskeletal protein (either a microtubule or actin filament, spindle pole body, or protein directly bound to them) and one or more other molecules, permitting them to function in a coordinated way. References: PMID:30323238 Sources: GOC:mtg_MIT_16mar07 Also known as: cytoskeletal adaptor activity Relationships: is a type of protein-macromolecule adaptor activity [GO:0030674]; has part cytoskeletal protein binding [GO:0008092] Subtypes: GO:0106006, spindle pole body anchor activity [GO:0140475]